positive regulation of fear response [GO:1903367] (biological process) Definition: Any process that activates or increases the frequency, rate or extent of fear response. Relationships: is a type of positive regulation of response to stimulus [GO:0048584]; is_a positive regulation of multicellular organismal process [GO:0051240]; is a type of regulation of fear response [GO:1903365]; positively regulates GO:0042596 Subtypes: positive regulation of behavioral fear response [GO:2000987] Also known as: positive regulation of physiological fear response, up regulation of fear response, up regulation of physiological fear response, up-regulation of fear response, up-regulation of physiological fear response, upregulation of fear response, upregulation of physiological fear response, activation of fear response, activation of physiological fear response References: PMID:8677262 Sources: GOC:TermGenie, GOC:mr, GO_REF:0000058